{
  "gene": "UniProtKB:O95049",
  "gene_name": "Tight junction protein ZO-3",
  "gene_symbol": "TJP3",
  "term_id": "GO:0150105",
  "term_label": "protein localization to cell-cell junction"
}